germ-line stem cell division [GO:0042078] (biological process) Subtypes: germline stem cell asymmetric division [GO:0098728], germline stem cell symmetric division [GO:0098729] References: PMID:2279698 Sources: GOC:jid Definition: The self-renewing division of a germline stem cell to produce a daughter stem cell and a daughter germ cell, which will divide to form the gametes. Also known as: germ-line stem cell renewal Relationships: is a type of GO:0017145; is part of germ cell development [GO:0007281]